aureusidin synthase activity [GO:0033793] (molecular function) Sources: EC:1.21.3.6 Relationships: is a type of oxidoreductase activity, acting on X-H and Y-H to form an X-Y bond, with oxygen as acceptor [GO:0046993] Definition: Catalysis of the reactions: 2',4,4',6'-tetrahydroxychalcone 4'-O-beta-D-glucoside + H+ + O2 = aureusidin 6-O-beta-glucoside + H2O, 2 2',3,4,4',6'-pentahydroxychalcone 4'-O-beta-D-glucoside + 2 H+ + O2 = 2 aureusidin 6-O-beta-glucoside + 2 H2O, and 2',3,4,4',6'-pentahydroxychalcone 4'-O-beta-D-glucoside + H+ + O2 = bracteatin 6-O-beta-glucoside + H2O. This activity consists of two separate chemical transformations: 3-hydroxylation and oxidative cyclization (2',-dehydrogenation). Also known as: 2',4,4',6'-tetrahydroxychalcone:oxygen oxidoreductase activity